regulation of 4,6-pyruvylated galactose residue biosynthetic process [GO:0060634] (biological process) Sources: GOC:dph, GOC:tb Definition: Any process that modulates the rate, frequency, or extent of 4,6-pyruvylated galactose residue biosynthetic process, the chemical reactions and pathways resulting in the formation of the pyruvylated galactose residue 4-6-O-[(R)(1-carboxyethylidine)]-Gal-beta-(1->3)-. The galactose residue is part of a larger polysaccharide chain. Relationships: is a type of regulation of polysaccharide biosynthetic process [GO:0032885]; regulates 4,6-pyruvylated galactose residue biosynthetic process [GO:0051072]